amine transport [GO:0015837] (BP) Definition: The directed movement of amines, including polyamines, organic compounds containing one or more amino groups, into, out of or within a cell, or between cells, by means of some agent such as a transporter or pore. Sources: GOC:ai, ISBN:0198506732 Also known as: amine/polyamine transport Relationships: is a type of nitrogen compound transport [GO:0071705] Subtypes: chromaffin granule amine transport [GO:0015841], aminergic neurotransmitter loading into synaptic vesicle [GO:0015842], methylammonium transport [GO:0015843], ethanolamine transport [GO:0034229], primary amine secretion [GO:0061531] Regulation: regulated by regulation of amine transport [GO:0051952]; negatively regulated by negative regulation of amine transport [GO:0051953]; positively regulated by positive regulation of amine transport [GO:0051954]